{
  "term_id": "GO:0019075",
  "gene_symbol": "MVB12B",
  "term_label": "virus maturation",
  "gene": "UniProtKB:Q9H7P6",
  "gene_name": "Multivesicular body subunit 12B"
}